{
  "term_id": "GO:0000981",
  "gene": "UniProtKB:O95780",
  "gene_name": "Zinc finger protein 682",
  "gene_symbol": "ZNF682",
  "term_label": "DNA-binding transcription factor activity, RNA polymerase II-specific"
}